{
  "term_id": "GO:0043434",
  "gene_symbol": "REG1B",
  "term_label": "response to peptide hormone",
  "gene_name": "Lithostathine-1-beta",
  "gene": "UniProtKB:P48304"
}